symbiont-mediated perturbation of host apoptosis [GO:0052150] (biological process) Subtypes: symbiont-mediated suppression of host apoptosis [GO:0033668], symbiont-mediated activation of host apoptosis [GO:0052151] Sources: GOC:curators Definition: A process in which a symbiont gene product affects host apoptosis, leading to a change in the frequency, rate or extent of apoptosis in the host cell. The host is defined as the larger of the organisms involved in a symbiotic interaction. Note: Note that term is to be used to annotate gene products in the symbiont. To annotate host gene products, consider the biological process term 'regulation of apoptosis ; GO:0042981'. Also known as: modulation by organism of host apoptotic programmed cell death, modulation by symbiont of host apoptotic process, modulation by symbiont of host apoptosis, modulation by virus of host apoptosis, regulation by virus of host apoptosis Relationships: is a type of GO:0051709; is a type of GO:0052040